{
  "term_id": "GO:0051604",
  "gene_name": "Lipase maturation factor 1",
  "gene_symbol": "LMF1",
  "term_label": "protein maturation",
  "gene": "UniProtKB:Q96S06"
}